deoxyribonucleoside triphosphate biosynthetic process [GO:0009202] (biological process) Subtypes: GO:0009216 Sources: GOC:go_curators, ISBN:0198506732 Also known as: deoxyribonucleoside triphosphate anabolism, deoxyribonucleoside triphosphate biosynthesis, deoxyribonucleoside triphosphate formation, deoxyribonucleoside triphosphate synthesis Definition: The chemical reactions and pathways resulting in the formation of a deoxyribonucleoside triphosphate, a compound consisting of a nucleobase linked to a deoxyribose sugar esterified with triphosphate on the sugar. Relationships: is a type of nucleoside triphosphate biosynthetic process [GO:0009142]; is a type of deoxyribonucleoside triphosphate metabolic process [GO:0009200]